{
  "term_id": "UNKNOWN:0001",
  "gene_name": "Phosphoribosyltransferase domain-containing protein 1",
  "gene_symbol": "PRTFDC1",
  "term_label": "Unknown molecular function",
  "gene": "UniProtKB:Q9NRG1"
}